short descending thin limb development [GO:0072063] (BP) Subtypes: GO:0072271 Relationships: is a type of nephron epithelium development [GO:0072009]; is a type of descending thin limb development [GO:0072022]; is part of short nephron development [GO:0072030] Definition: The process whose specific outcome is the progression of the short descending thin limb over time, from its formation to the mature structure. The short descending thin limb is the descending thin limb of a short nephron that has a squamous epithelial morphology. Sources: GOC:mtg_kidney_jan10